{
  "gene_name": "Cytosolic 5'-nucleotidase 3A",
  "term_id": "GO:0005737",
  "gene": "UniProtKB:Q9H0P0",
  "term_label": "cytoplasm",
  "gene_symbol": "NT5C3A"
}